{
  "term_id": "GO:0022848",
  "term_label": "acetylcholine-gated monoatomic cation-selective channel activity",
  "gene_symbol": "CHRNG",
  "gene_name": "Acetylcholine receptor subunit gamma",
  "gene": "UniProtKB:P07510"
}